{
  "term_label": "innate immune response",
  "gene_name": "Ret finger protein-like 2",
  "gene_symbol": "RFPL2",
  "term_id": "GO:0045087",
  "gene": "UniProtKB:O75678"
}